{
  "gene": "UniProtKB:Q6ZUF6",
  "term_id": "UNKNOWN:0003",
  "gene_symbol": "LINC00336",
  "term_label": "Unknown cellular component",
  "gene_name": "Putative uncharacterized protein encoded by LINC00336"
}